phosphorylation [GO:0016310] (biological process) Subtypes: glucose 1-phosphate phosphorylation [GO:0006009], protein phosphorylation [GO:0006468], photosynthetic phosphorylation [GO:0009777], organic acid phosphorylation [GO:0031388], lipid phosphorylation [GO:0046834], GO:0046835 Relationships: is a type of phosphate-containing compound metabolic process [GO:0006796] Definition: The process of introducing a phosphate group into a molecule, usually with the formation of a phosphoric ester, a phosphoric anhydride or a phosphoric amide. Sources: ISBN:0198506732 Regulation: regulated by regulation of phosphorylation [GO:0042325]; RO_0002212 by negative regulation of phosphorylation [GO:0042326]; positively regulated by GO:0042327